{
  "gene_name": "Thioredoxin domain-containing protein 16",
  "term_id": "UNKNOWN:0002",
  "gene": "UniProtKB:Q9P2K2",
  "gene_symbol": "TXNDC16",
  "term_label": "Unknown biological process"
}